positive regulation of norepinephrine uptake [GO:0051623] (biological process) Definition: Any process that activates or increases the frequency, rate or extent of the directed movement of norepinephrine into a cell. Sources: GOC:ai Relationships: is a type of positive regulation of transport [GO:0051050]; is a type of GO:0051621; positively regulates norepinephrine uptake [GO:0051620] Also known as: positive regulation of levarterenol uptake, positive regulation of noradrenaline uptake, positive regulation of norepinephrine import, up regulation of norepinephrine uptake, up-regulation of norepinephrine uptake, upregulation of norepinephrine uptake, activation of norepinephrine uptake, stimulation of norepinephrine uptake